{
  "gene_symbol": "FAM227A",
  "gene": "UniProtKB:F5H4B4",
  "term_label": "Unknown biological process",
  "gene_name": "Protein FAM227A",
  "term_id": "UNKNOWN:0002"
}